{
  "term_label": "enzyme regulator activity",
  "gene": "UniProtKB:P12074",
  "term_id": "GO:0030234",
  "gene_name": "Cytochrome c oxidase subunit 6A1, mitochondrial",
  "gene_symbol": "COX6A1"
}